negative regulation of T-helper 17 cell extravasation [GO:2000456] (biological process) Relationships: is a type of negative regulation of CD8-positive, alpha-beta T cell extravasation [GO:2000450]; is a type of regulation of T-helper 17 cell extravasation [GO:2000455]; negatively regulates T-helper 17 cell extravasation [GO:0035699] Definition: Any process that stops, prevents or reduces the frequency, rate or extent of T-helper 17 cell extravasation. Sources: GOC:obol